{
  "gene_name": "Alpha-ketoglutarate-dependent dioxygenase FTO",
  "term_id": "GO:0035516",
  "term_label": "broad specificity oxidative DNA demethylase activity",
  "gene": "UniProtKB:Q9C0B1",
  "gene_symbol": "FTO"
}